negative regulation of asymmetric cell division [GO:0045769] (BP) Also known as: down regulation of asymmetric cell division, down-regulation of asymmetric cell division, downregulation of asymmetric cell division, inhibition of asymmetric cell division Subtypes: GO:1904839, negative regulation of establishment or maintenance of neuroblast polarity [GO:2000248] Definition: Any process that stops, prevents, or reduces the frequency, rate or extent of asymmetric cell division. Relationships: is a type of regulation of asymmetric cell division [GO:0009786]; is a type of GO:0051782; negatively regulates asymmetric cell division [GO:0008356] Sources: GOC:go_curators